hexosyltransferase activity [GO:0016758] (molecular function) Relationships: is a type of glycosyltransferase activity [GO:0016757] Definition: Catalysis of the transfer of a hexosyl group from one compound (donor) to another (acceptor). Also known as: transferase activity, transferring hexosyl groups Sources: EC:2.4.1.- Subtypes: mannosyltransferase activity [GO:0000030], mannosylphosphate transferase activity [GO:0000031], 1,4-alpha-glucan branching enzyme activity [GO:0003844], 4-alpha-glucanotransferase activity [GO:0004134], oligosaccharyl transferase activity [GO:0004576], 1,4-alpha-oligoglucan phosphorylase activity [GO:0004645], acetylglucosaminyltransferase activity [GO:0008375], acetylgalactosaminyltransferase activity [GO:0008376], galactosyltransferase activity [GO:0008378], fucosyltransferase activity [GO:0008417], O antigen polymerase activity [GO:0008755], lipid-A-disaccharide synthase activity [GO:0008915], peptidoglycan glycosyltransferase activity [GO:0008955], GO:0015020, phenanthrol glycosyltransferase activity [GO:0019112], GO:0033834, flavanone 7-O-glucoside 2''-O-beta-L-rhamnosyltransferase activity [GO:0033835], phosphatidylinositol alpha-mannosyltransferase activity [GO:0043750], GO:0043895, GO:0045140, GO:0046510, glucosyltransferase activity [GO:0046527], alpha-1,4-glucan-protein synthase (ADP-forming) activity [GO:0047211], flavonol-3-O-glucoside L-rhamnosyltransferase activity [GO:0047230], GO:0047244, diglucosyl diacylglycerol synthase activity [GO:0047257], alpha,alpha-trehalose-phosphate synthase (GDP-forming) activity [GO:0047260], polygalacturonate 4-alpha-galacturonosyltransferase activity [GO:0047262], GO:0047514, 1,3-beta-oligoglucan phosphorylase activity [GO:0047515], abequosyltransferase activity [GO:0047600], alginate synthase activity [GO:0047643], alpha-1,3-glucan synthase activity [GO:0047657], amylosucrase activity [GO:0047669], GO:0047725, dextransucrase activity [GO:0047849], laminaribiose phosphorylase activity [GO:0050045], GO:0050053, linamarin synthase activity [GO:0050057], GO:0050102, dextrin dextranase activity [GO:0050103], GO:0050420, 1,3-beta-galactosyl-N-acetylhexosamine phosphorylase activity [GO:0050500], GO:0050501, mannosyl-3-phosphoglycerate synthase activity [GO:0050504], fructosyltransferase activity [GO:0050738], anthocyanidin 3-glucoside rhamnosyltransferase activity [GO:0051566], 4-acetamido-4,6-dideoxy-D-galactose transferase activity [GO:0102031], decaprenyl-N-acetyl-alpha-D-glucosaminyl-pyrophosphate:dTDP-alpha-L-rhamnose rhamnosyltransferase activity [GO:0102096], GO:0102159, cyanidin 3-O-glucoside 2-O-glucuronosyltransferase activity [GO:0102160], GO:0102240, soyasaponin III rhamnosyltransferase activity [GO:0102241], 2-deoxystreptamine glucosyltransferase activity [GO:0102318], 2-deoxystreptamine N-acetyl-D-glucosaminyltransferase activity [GO:0102319], N,N'-diacetylbacillosaminyl-diphospho-undecaprenol alpha-1,3-N-acetylgalactosaminyltransferase activity [GO:0102335], steviol 13-O glucosyltransferase activity [GO:0102377], steviolmonoside glucosyltransferase activity [GO:0102378], steviolbioside glucosyltransferase activity (stevioside forming) [GO:0102379], steviolbioside glucosyltransferase activity (rebaudioside B forming) [GO:0102380], GO:0102381, rebaudioside B glucosyltransferase activity [GO:0102382], (+)-sesaminol 2-O-glucosyltransferase activity [GO:0102423], cyanidin 3-O-galactosyltransferase activity [GO:0102454], anthocyanidin 3-O-glucoside 2''-O-glucosyltransferase activity [GO:0102455], cyanidin 3-O-glucoside 7-O-glucosyltransferase (acyl-glucose) activity [GO:0102457], scutellarein 7-O-glucuronosyltransferase activity [GO:0102467], wogonin 7-O-glucuronosyltransferase activity [GO:0102468], cyanidin 3-O-glucoside 5-O-glucosyltransferase (acyl-glucose) activity [GO:0102506], (+)-secoisolariciresinol glucosyltransferase activity [GO:0102610], (+)-secoisolariciresinol monoglucoside glucosyltransferase activity [GO:0102611], GO:0102710, soyasapogenol B glucuronosyltransferase activity [GO:0102793], GO:0102816, verbascose synthase activity [GO:0102830], stachyose synthase activity [GO:0102831], GO:0102832, chalcone 4'-O-glucosyltransferase activity [GO:0102890], UDPG:cyclo-DOPA 5-O-glucosyltransferase activity [GO:0102894], mannosylglycerate synthase activity [GO:0102921], GO:0102937, 1,2-rhamnosyltransferase activity [GO:0102949], 7-deoxyloganetic acid glucosyltransferase activity [GO:0102970], trehalose synthase activity [GO:0102986], mannosylfructose-phosphate synthase activity [GO:0103011], GO:0120514